positive regulation of epithelial cell differentiation involved in kidney development [GO:2000698] (biological process) Sources: GOC:mtg_kidney_jan10, GOC:yaf Relationships: is a type of positive regulation of epithelial cell differentiation [GO:0030858]; is_a regulation of epithelial cell differentiation involved in kidney development [GO:2000696]; positively regulates GO:0035850 Definition: Any process that activates or increases the frequency, rate or extent of epithelial cell differentiation involved in kidney development. Subtypes: positive regulation of mesenchymal to epithelial transition involved in metanephros morphogenesis [GO:0072108], GO:2000086, positive regulation of nephron tubule epithelial cell differentiation [GO:2000768]